{
  "term_id": "GO:0000151",
  "gene": "UniProtKB:Q9BSL1",
  "gene_symbol": "UBAC1",
  "term_label": "ubiquitin ligase complex",
  "gene_name": "Ubiquitin-associated domain-containing protein 1"
}